{
  "gene_name": "WD repeat-containing protein 17",
  "term_label": "Unknown molecular function",
  "gene_symbol": "WDR17",
  "term_id": "UNKNOWN:0001",
  "gene": "UniProtKB:Q8IZU2"
}